{
  "gene_name": "Interleukin-8",
  "term_label": "CXCR chemokine receptor binding",
  "term_id": "GO:0045236",
  "gene": "UniProtKB:P10145",
  "gene_symbol": "CXCL8"
}